1,2-dihydroxynaphthalene dioxygenase activity [GO:0018554] (molecular function) Definition: Catalysis of the reaction: 1,2-dihydroxynaphthalene + O2 = 2-hydroxychromene-2-carboxylate. C6 of the substrate molecular may have an NH2 group attached. Relationships: is a type of GO:0016701; is_a dioxygenase activity [GO:0051213] Sources: UM-BBD_enzymeID:r0336